{
  "gene_name": "DnaJ homolog subfamily B member 4",
  "term_id": "GO:0000122",
  "gene": "UniProtKB:Q9UDY4",
  "term_label": "negative regulation of transcription by RNA polymerase II",
  "gene_symbol": "DNAJB4"
}